{
  "term_label": "positive regulation of transcription by RNA polymerase II",
  "gene_name": "Nuclear factor of activated T-cells, cytoplasmic 2",
  "gene_symbol": "NFATC2",
  "gene": "UniProtKB:Q13469",
  "term_id": "GO:0045944"
}